negative regulation of plus-end directed microtubule sliding [GO:0062168] (biological process) Relationships: is a type of negative regulation of cellular process [GO:0048523]; is a type of regulation of plus-end directed microtubule sliding [GO:0062169]; negatively regulates GO:0031535 Definition: Any process that stops, prevents, or reduces the frequency, rate, or extent of plus-end directed microtubule sliding. References: PMID:21892183